{
  "term_label": "Unknown cellular component",
  "gene": "UniProtKB:Q9NRM6",
  "gene_symbol": "IL17RB",
  "term_id": "UNKNOWN:0003",
  "gene_name": "Interleukin-17 receptor B"
}